{
  "term_label": "Unknown biological process",
  "term_id": "UNKNOWN:0002",
  "gene_name": "Tripartite motif-containing protein 29",
  "gene": "UniProtKB:Q14134",
  "gene_symbol": "TRIM29"
}